endocytic vesicle [GO:0030139] (cellular component) References: PMID:19696797 Sources: GOC:go_curators Also known as: endocytotic transport vesicle, endocytotic vesicle Subtypes: post-lysosomal vacuole [GO:0032195], symbiosome [GO:0043659], clathrin-coated endocytic vesicle [GO:0045334], phagocytic vesicle [GO:0045335] Relationships: is a type of cytoplasmic vesicle [GO:0031410] Definition: A membrane-bounded intracellular vesicle formed by invagination of the plasma membrane around an extracellular substance. Endocytic vesicles fuse with early endosomes to deliver the cargo for further sorting.